negative regulation of myoblast proliferation [GO:2000818] (biological process) Subtypes: negative regulation of cardiac muscle myoblast proliferation [GO:0110023] Definition: Any process that stops, prevents or reduces the frequency, rate or extent of myoblast proliferation. Sources: GOC:obol Relationships: is a type of negative regulation of cell population proliferation [GO:0008285]; is a type of GO:2000291; negatively regulates GO:0051450